{
  "gene_symbol": "TTC12",
  "term_label": "axonemal dynein complex assembly",
  "gene_name": "Tetratricopeptide repeat protein 12",
  "gene": "UniProtKB:Q9H892",
  "term_id": "GO:0070286"
}